{
  "term_label": "Unknown cellular component",
  "gene_name": "S-adenosylmethionine sensor upstream of mTORC1",
  "term_id": "UNKNOWN:0003",
  "gene": "UniProtKB:Q1RMZ1",
  "gene_symbol": "BMT2"
}